{
  "term_id": "GO:0000981",
  "term_label": "DNA-binding transcription factor activity, RNA polymerase II-specific",
  "gene": "UniProtKB:Q8N1L9",
  "gene_symbol": "BATF2",
  "gene_name": "Basic leucine zipper transcriptional factor ATF-like 2"
}